{
  "term_label": "Unknown biological process",
  "gene_symbol": "FAM25C",
  "gene": "UniProtKB:B3EWG5",
  "gene_name": "Protein FAM25C",
  "term_id": "UNKNOWN:0002"
}